{
  "term_label": "epithelial cell differentiation",
  "term_id": "GO:0030855",
  "gene": "UniProtKB:Q99456",
  "gene_symbol": "KRT12",
  "gene_name": "Keratin, type I cytoskeletal 12"
}